regulation of synaptic vesicle uncoating [GO:1903388] (biological process) Also known as: regulation of synaptic vesicle coat depolymerization, regulation of synaptic vesicle coat protein depolymerization Definition: Any process that modulates the frequency, rate or extent of synaptic vesicle uncoating. Subtypes: negative regulation of synaptic vesicle uncoating [GO:1903389], positive regulation of synaptic vesicle uncoating [GO:1903390] References: PMID:21563316 Sources: GOC:PARL, GOC:TermGenie, GOC:pad, GO_REF:0000058 Relationships: is a type of GO:1901879; regulates synaptic vesicle uncoating [GO:0016191]